{
  "term_id": "UNKNOWN:0001",
  "term_label": "Unknown molecular function",
  "gene": "UniProtKB:A4QMS7",
  "gene_symbol": "CFAP90",
  "gene_name": "Cilia- and flagella-associated protein 90"
}